{
  "gene_symbol": "SSTR4",
  "gene_name": "Somatostatin receptor type 4",
  "term_id": "GO:0043005",
  "term_label": "neuron projection",
  "gene": "UniProtKB:P31391"
}